regulation of serotonin biosynthetic process [GO:1905627] (biological process) References: PMID:25642596 Sources: GOC:PARL, GOC:TermGenie, GOC:pad, GO_REF:0000058 Also known as: regulation of serotonin anabolism, regulation of serotonin biosynthesis, regulation of serotonin formation, regulation of serotonin synthesis Subtypes: negative regulation of serotonin biosynthetic process [GO:1905628], positive regulation of serotonin biosynthetic process [GO:1905629] Relationships: is_a regulation of biosynthetic process [GO:0009889]; regulates serotonin biosynthetic process [GO:0042427] Definition: Any process that modulates the frequency, rate or extent of serotonin biosynthetic process.